{
  "term_label": "signal transduction",
  "term_id": "GO:0007165",
  "gene_name": "T-complex protein 11-like protein 2",
  "gene_symbol": "TCP11L2",
  "gene": "UniProtKB:Q8N4U5"
}